{
  "gene_symbol": "FOXE1",
  "term_label": "anatomical structure morphogenesis",
  "gene_name": "Forkhead box protein E1",
  "term_id": "GO:0009653",
  "gene": "UniProtKB:O00358"
}